{
  "gene_symbol": "LDHB",
  "gene_name": "L-lactate dehydrogenase B chain",
  "term_id": "GO:0005739",
  "gene": "UniProtKB:P07195",
  "term_label": "mitochondrion"
}